{
  "term_label": "Unknown molecular function",
  "gene_name": "Proliferation-associated protein 2G4",
  "gene_symbol": "PA2G4",
  "gene": "UniProtKB:Q9UQ80",
  "term_id": "UNKNOWN:0001"
}